{
  "gene_symbol": "LRP4",
  "gene": "UniProtKB:O75096",
  "term_label": "synapse organization",
  "term_id": "GO:0050808",
  "gene_name": "Low-density lipoprotein receptor-related protein 4"
}